phenol beta-glucosyltransferase activity [GO:0050171] (molecular function) Also known as: phenol b-glucosyltransferase activity, UDP glucosyltransferase activity, UDP-glucose glucosyltransferase activity, UDP-glucose:phenol beta-D-glucosyltransferase activity, UDPglucose:phenol beta-D-glucosyltransferase activity, UDPglucosyltransferase activity, phenol-beta-D-glucosyltransferase activity, uridine diphosphoglucosyltransferase activity Definition: Catalysis of the reaction: UDP-glucose + a phenol = UDP + an aryl beta-D-glucoside. Sources: EC:2.4.1.35, MetaCyc:PHENOL-BETA-GLUCOSYLTRANSFERASE-RXN Relationships: is a type of UDP-glucosyltransferase activity [GO:0035251]